{
  "gene": "UniProtKB:P56199",
  "gene_name": "Integrin alpha-1",
  "gene_symbol": "ITGA1",
  "term_label": "integrin-mediated signaling pathway",
  "term_id": "GO:0007229"
}